{
  "term_id": "GO:0043328",
  "gene": "UniProtKB:Q92783",
  "gene_name": "Signal transducing adapter molecule 1",
  "term_label": "protein transport to vacuole involved in ubiquitin-dependent protein catabolic process via the multivesicular body sorting pathway",
  "gene_symbol": "STAM"
}